{
  "term_label": "RNA binding",
  "gene": "UniProtKB:Q96AK3",
  "gene_name": "DNA dC-dU-editing enzyme APOBEC-3D",
  "gene_symbol": "APOBEC3D",
  "term_id": "GO:0003723"
}